{
  "term_label": "box C/D snoRNP assembly",
  "gene_symbol": "ZNHIT3",
  "gene_name": "Zinc finger HIT domain-containing protein 3",
  "term_id": "GO:0000492",
  "gene": "UniProtKB:Q15649"
}